regulation of determination of dorsal identity [GO:2000015] (biological process) Also known as: regulation of determination of adaxial identity Definition: Any process that modulates the frequency, rate or extent of determination of dorsal identity. Relationships: is a type of regulation of multicellular organismal process [GO:0051239]; regulates determination of dorsal identity [GO:0048263] Sources: GOC:obol Subtypes: negative regulation of determination of dorsal identity [GO:2000016], positive regulation of determination of dorsal identity [GO:2000017]